{
  "gene": "UniProtKB:Q14008",
  "gene_name": "Cytoskeleton-associated protein 5",
  "term_label": "microtubule plus-end",
  "gene_symbol": "CKAP5",
  "term_id": "GO:0035371"
}